{
  "gene": "UniProtKB:Q4G0X9",
  "term_label": "cytoplasm",
  "gene_symbol": "CCDC40",
  "term_id": "GO:0005737",
  "gene_name": "Coiled-coil domain-containing protein 40"
}